response to light stimulus [GO:0009416] (biological process) Subtypes: visual behavior [GO:0007632], response to UV [GO:0009411], detection of light stimulus [GO:0009583], response to blue light [GO:0009637], response to red or far red light [GO:0009639], response to light intensity [GO:0009642], photoperiodism [GO:0009648], GO:0009704, photoprotection [GO:0010117], cone photoresponse recovery [GO:0036368], phototaxis [GO:0042331], cellular response to light stimulus [GO:0071482], energy quenching [GO:1990066] Sources: GOC:go_curators, ISBN:0582227089 Definition: Any process that results in a change in state or activity of a cell or an organism (in terms of movement, secretion, enzyme production, gene expression, etc.) as a result of a light stimulus, electromagnetic radiation of wavelengths classified as infrared, visible or ultraviolet light. Relationships: is a type of response to radiation [GO:0009314]